{
  "term_label": "guanyl-nucleotide exchange factor activity",
  "gene_symbol": "VAV2",
  "gene": "UniProtKB:P52735",
  "term_id": "GO:0005085",
  "gene_name": "Guanine nucleotide exchange factor VAV2"
}